leukocyte chemotaxis [GO:0030595] (BP) Sources: GOC:add, GOC:jl Subtypes: leukocyte chemotaxis involved in inflammatory response [GO:0002232], leukocyte chemotaxis involved in immune response [GO:0002233], dendritic cell chemotaxis [GO:0002407], monocyte chemotaxis [GO:0002548], mast cell chemotaxis [GO:0002551], macrophage chemotaxis [GO:0048246], GO:0048247, granulocyte chemotaxis [GO:0071621] Definition: The movement of a leukocyte in response to an external stimulus. Relationships: is a type of leukocyte migration [GO:0050900]; is a type of cell chemotaxis [GO:0060326] Also known as: immune cell chemotaxis, leucocyte chemotaxis Regulation: regulated by GO:0002688; negatively regulated by negative regulation of leukocyte chemotaxis [GO:0002689]; positively regulated by positive regulation of leukocyte chemotaxis [GO:0002690]